negative regulation of RNA biosynthetic process [GO:1902679] (biological process) Definition: Any process that stops, prevents or reduces the frequency, rate or extent of RNA biosynthetic process. Subtypes: GO:0045869, negative regulation of DNA-templated transcription [GO:0045892], negative regulation of promoter clearance from RNA polymerase II promoter [GO:0140847] Also known as: down regulation of RNA anabolism, down regulation of RNA biosynthesis, down regulation of RNA biosynthetic process, down regulation of RNA formation, down regulation of RNA synthesis, down-regulation of RNA anabolism, down-regulation of RNA biosynthesis, down-regulation of RNA biosynthetic process, down-regulation of RNA formation, down-regulation of RNA synthesis, downregulation of RNA anabolism, downregulation of RNA biosynthesis, downregulation of RNA biosynthetic process, downregulation of RNA formation, downregulation of RNA synthesis, negative regulation of RNA anabolism, negative regulation of RNA biosynthesis, negative regulation of RNA formation, negative regulation of RNA synthesis, inhibition of RNA anabolism, inhibition of RNA biosynthesis, inhibition of RNA biosynthetic process, inhibition of RNA formation, inhibition of RNA synthesis Relationships: is a type of negative regulation of macromolecule biosynthetic process [GO:0010558]; is a type of negative regulation of RNA metabolic process [GO:0051253]; is_a GO:2001141; negatively regulates RNA biosynthetic process [GO:0032774] Sources: GO:jl, GOC:TermGenie, GO_REF:0000058